L-tryptophan catabolic process to indole-3-acetate [GO:0019440] (biological process) Definition: The chemical reactions and pathways resulting in the breakdown of L-tryptophan into other compounds, including indole-3-acetate. Sources: GOC:go_curators Also known as: tryptophan breakdown to indole-3-acetate, tryptophan catabolic process to IAA, tryptophan catabolic process to indole-3-acetate, tryptophan catabolic process to indoleacetic acid, tryptophan catabolism to indoleacetic acid, tryptophan degradation to indole-3-acetate Relationships: is_a L-tryptophan catabolic process [GO:0006569]; is a type of monocarboxylic acid metabolic process [GO:0032787]